septin complex [GO:0031105] (cellular component) Subtypes: mitotic septin complex [GO:0032151], meiotic septin complex [GO:0032152] Relationships: is a type of GO:0032991; is part of cell cortex [GO:0005938]; is part of septin cytoskeleton [GO:0032156] Definition: A protein complex containing septins. Typically, these complexes contain multiple septins and are oligomeric. References: PMID:15385632 Sources: GOC:mah